{
  "gene_symbol": "HTR3C",
  "gene": "UniProtKB:Q8WXA8",
  "gene_name": "5-hydroxytryptamine receptor 3C",
  "term_id": "GO:0005886",
  "term_label": "plasma membrane"
}